capsule [GO:0042603] (cellular component) Definition: A protective structure surrounding some fungi and bacteria, attached externally to the cell wall and composed primarily of polysaccharides. Capsules are highly organized structures that adhere strongly to cells and cannot be easily removed. Capsules play important roles in pathogenicity, preventing phagocytosis by other cells, adherence, and resistance to desiccation. Relationships: is a type of glycocalyx [GO:0030112] Sources: GOC:mlg